{
  "gene_symbol": "RCAN2",
  "gene_name": "Calcipressin-2",
  "term_label": "nucleus",
  "gene": "UniProtKB:Q14206",
  "term_id": "GO:0005634"
}